cellular response to antimycin A [GO:0072745] (biological process) Definition: Any process that results in a change in state or activity of a cell (in terms of movement, secretion, enzyme production, gene expression, etc.) as a result of an antimycin A stimulus. Sources: GOC:mah Relationships: is a type of response to antimycin A [GO:1901325]; is_a cellular response to nitrogen compound [GO:1901699]; is a type of cellular response to oxygen-containing compound [GO:1901701]